{
  "gene_symbol": "ODAD1",
  "gene_name": "Outer dynein arm-docking complex subunit 1",
  "term_label": "axoneme",
  "term_id": "GO:0005930",
  "gene": "UniProtKB:Q96M63"
}